{
  "gene_symbol": "SNAP23",
  "gene_name": "Synaptosomal-associated protein 23",
  "gene": "UniProtKB:O00161",
  "term_label": "synaptic vesicle priming",
  "term_id": "GO:0016082"
}